GABA receptor binding [GO:0050811] (MF) Definition: Binding to a gamma-aminobutyric acid (GABA, 4-aminobutyrate) receptor. Also known as: 4-aminobutanoate receptor binding, 4-aminobutyrate receptor binding, gamma-aminobutyric acid receptor binding, diazepam binding inhibitor activity Subtypes: G protein-coupled GABA receptor binding [GO:0031795] Sources: GOC:ai Relationships: is a type of GO:0005102